{
  "term_label": "endoplasmic reticulum",
  "term_id": "GO:0005783",
  "gene_symbol": "CES1P1",
  "gene": "UniProtKB:Q9UKY3",
  "gene_name": "Putative inactive carboxylesterase 4"
}